{
  "term_label": "plasma membrane",
  "term_id": "GO:0005886",
  "gene_name": "Agrin",
  "gene": "UniProtKB:O00468",
  "gene_symbol": "AGRN"
}